{
  "term_label": "ribonucleoprotein complex",
  "gene_name": "CUGBP Elav-like family member 3",
  "gene": "UniProtKB:Q5SZQ8",
  "term_id": "GO:1990904",
  "gene_symbol": "CELF3"
}